tannase activity [GO:0050318] (molecular function) Also known as: tannase S, tannin acetylhydrolase activity, tannin acylhydrolase activity Sources: EC:3.1.1.20, RHEA:16365 Relationships: is a type of GO:0052689 Definition: Catalysis of the reaction: digallate + H2O = 2 gallate + H+.